{
  "gene_name": "Forkhead box protein F2",
  "gene": "UniProtKB:Q12947",
  "term_id": "GO:0009887",
  "gene_symbol": "FOXF2",
  "term_label": "animal organ morphogenesis"
}